glucosamine 6-phosphate N-acetyltransferase activity [GO:0004343] (molecular function) Also known as: glucosamine-phosphate N-acetyltransferase activity, D-glucosamine-6-P N-acetyltransferase activity, N-acetylglucosamine-6-phosphate synthase activity, acetyl-CoA:D-glucosamine-6-phosphate N-acetyltransferase activity, aminodeoxyglucosephosphate acetyltransferase activity, glucosamine 6-phosphate acetylase activity, glucosamine-6-phosphate acetylase activity, phosphoglucosamine N-acetylase activity, phosphoglucosamine acetylase activity, phosphoglucosamine transacetylase activity Sources: EC:2.3.1.4, RHEA:10292 Relationships: is a type of N-acetyltransferase activity [GO:0008080] Definition: Catalysis of the reaction: D-glucosamine 6-phosphate + acetyl-CoA = N-acetyl-D-glucosamine 6-phosphate + CoA + H+.